response to anticonvulsant [GO:0036277] (biological process) Relationships: is a type of response to chemical [GO:0042221] Definition: Any process that results in a change in state or activity of a cell or an organism (in terms of movement, secretion, enzyme production, gene expression, etc.) as a result of an anticonvulsant stimulus, a drug used to prevent seizures or reduce their severity. Note: Note that this term is in the subset of terms that should not be used for direct manual annotation of gene products. It was created to be used for cross-referencing by other ontologies. Direct annotations to this term may be amended during annotation QC. Sources: GOC:hp